{
  "gene_name": "Tyrosine-protein kinase transmembrane receptor ROR2",
  "term_id": "GO:0007169",
  "gene_symbol": "ROR2",
  "gene": "UniProtKB:Q01974",
  "term_label": "cell surface receptor protein tyrosine kinase signaling pathway"
}